{
  "term_label": "Unknown biological process",
  "gene_name": "Olfactory receptor 52A1",
  "gene_symbol": "OR52A1",
  "term_id": "UNKNOWN:0002",
  "gene": "UniProtKB:Q9UKL2"
}